2-hydroxyflavanone C-glucosyltransferase activity [GO:0120514] (molecular function) Relationships: is a type of hexosyltransferase activity [GO:0016758] Definition: Catalysis of the reaction: a 3'-hydro-2'-hydroxy-beta-oxodihydrochalcone + UDP-alpha-D-glucose = a 3'-(beta-D-glucopyranosyl)-2'-hydroxy-beta-oxodihydrochalcone + H+ + UDP. Sources: RHEA:51504